detection of mechanical stimulus involved in sensory perception of sound [GO:0050910] (biological process) Definition: The series of events involved in the perception of sound vibration in which the vibration is received and converted into a molecular signal. Sources: GOC:ai Also known as: detection of sound, hearing, sensory transduction of sound, perception of sound, detection of mechanical stimulus, perception of sound, sensory detection of mechanical stimulus, perception of sound, sensory transduction of mechanical stimulus, sensory detection of mechanical stimulus during perception of sound, sensory transduction of mechanical stimulus during perception of sound, sensory transduction of sound Relationships: is a type of nervous system process [GO:0050877]; is a type of GO:0050974; is part of sensory perception of sound [GO:0007605]